positive regulation of abscisic acid-activated signaling pathway [GO:0009789] (biological process) Definition: Any process that activates or increases the frequency, rate or extent of abscisic acid (ABA) signaling. Sources: GOC:lr Also known as: positive regulation of abscisic acid mediated signalling, up regulation of abscisic acid mediated signaling, up-regulation of abscisic acid mediated signaling, upregulation of abscisic acid mediated signaling, activation of abscisic acid mediated signaling, stimulation of abscisic acid mediated signaling, positive regulation of abscisic acid mediated signaling pathway Relationships: is_a regulation of abscisic acid-activated signaling pathway [GO:0009787]; is a type of GO:0009967; positively regulates abscisic acid-activated signaling pathway [GO:0009738]